{
  "gene_symbol": "SGCG",
  "gene_name": "Gamma-sarcoglycan",
  "gene": "UniProtKB:Q13326",
  "term_label": "sarcoglycan complex",
  "term_id": "GO:0016012"
}